phosphofructokinase activity [GO:0008443] (molecular function) Definition: Catalysis of the transfer of a phosphate group, usually from ATP, to a phosphofructose substrate molecule. Sources: GOC:jl Relationships: is a type of phosphotransferase activity, alcohol group as acceptor [GO:0016773]; is a type of carbohydrate kinase activity [GO:0019200] Subtypes: 6-phosphofructokinase activity [GO:0003872], 6-phosphofructo-2-kinase activity [GO:0003873], 1-phosphofructokinase activity [GO:0008662], GO:0047334